{
  "gene_symbol": "RANBP2",
  "term_label": "NLS-bearing protein import into nucleus",
  "term_id": "GO:0006607",
  "gene_name": "E3 SUMO-protein ligase RanBP2",
  "gene": "UniProtKB:P49792"
}